{
  "term_label": "fatty acid beta-oxidation using acyl-CoA dehydrogenase",
  "term_id": "GO:0033539",
  "gene_name": "Electron transfer flavoprotein subunit beta",
  "gene": "UniProtKB:P38117",
  "gene_symbol": "ETFB"
}